{
  "gene_symbol": "MLH1",
  "gene": "UniProtKB:P40692",
  "gene_name": "DNA mismatch repair protein Mlh1",
  "term_label": "ATP hydrolysis activity",
  "term_id": "GO:0016887"
}